cellular response to progesterone stimulus [GO:0071393] (biological process) Sources: GOC:mah Definition: Any process that results in a change in state or activity of a cell (in terms of movement, secretion, enzyme production, gene expression, etc.) as a result of a progesterone stimulus. Relationships: is a type of response to progesterone [GO:0032570]; is a type of cellular response to steroid hormone stimulus [GO:0071383]; is a type of cellular response to ketone [GO:1901655]